rhamnetin 3'-O-methyltransferase activity [GO:0102447] (molecular function) Sources: RHEA:73271 Definition: Catalysis of the reaction: rhamnetin + S-adenosyl-L-methionine = H+ + rhamnacene + S-adenosyl-L-homocysteine. Relationships: is_a methyltransferase activity [GO:0008168]